{
  "gene_symbol": "MT1B",
  "gene_name": "Metallothionein-1B",
  "term_id": "GO:0071276",
  "term_label": "cellular response to cadmium ion",
  "gene": "UniProtKB:P07438"
}